{
  "term_label": "lipopeptide binding",
  "gene_symbol": "CD1E",
  "gene_name": "T-cell surface glycoprotein CD1e, membrane-associated",
  "gene": "UniProtKB:P15812",
  "term_id": "GO:0071723"
}